regulation of defecation rhythm [GO:2000746] (biological process) Subtypes: negative regulation of defecation rhythm [GO:2000747], positive regulation of defecation rhythm [GO:2000748] Also known as: regulation of DMP, regulation of defecation cycle, regulation of defecation motor program, regulation of defecation behavior Sources: GOC:kmv Definition: Any process that modulates the frequency, rate or extent of defecation rhythm. Relationships: is a type of GO:2000292; regulates GO:0035882